post-embryonic anal fin morphogenesis [GO:0035135] (biological process) Definition: The process, occurring after embryonic development, by which the anatomical structures of the anal fin are generated and organized. An anal fin is an unpaired medial fin on the ventral aspect near the caudal end of a fish, which provides lateral stability while swimming. Relationships: is a type of post-embryonic medial fin morphogenesis [GO:0035132]; is_a anal fin morphogenesis [GO:0035144] Sources: GOC:dgh